{
  "gene": "UniProtKB:Q7LBR1",
  "term_id": "GO:0032509",
  "term_label": "endosome transport via multivesicular body sorting pathway",
  "gene_name": "Charged multivesicular body protein 1b",
  "gene_symbol": "CHMP1B"
}